depsipeptide metabolic process [GO:0050761] (biological process) Also known as: depsipeptide metabolism Subtypes: GO:0050762, depsipeptide biosynthetic process [GO:0050763] Relationships: is_a amide metabolic process [GO:0043603] Definition: The chemical reactions and pathways involving depsipeptides, a linear or cyclic compound composed of both amino acids and hydroxy acids in peptide and ester bonds respectively. Sources: GOC:go_curators